{
  "gene_symbol": "TENM2",
  "gene_name": "Teneurin-2",
  "gene": "UniProtKB:Q9NT68",
  "term_label": "neuron projection",
  "term_id": "GO:0043005"
}